{
  "gene_symbol": "LCTL",
  "term_id": "UNKNOWN:0002",
  "term_label": "Unknown biological process",
  "gene_name": "Lactase-like protein",
  "gene": "UniProtKB:Q6UWM7"
}